{
  "gene_name": "Transcription factor E2F4",
  "gene": "UniProtKB:Q16254",
  "term_id": "GO:0090575",
  "term_label": "RNA polymerase II transcription regulator complex",
  "gene_symbol": "E2F4"
}